{
  "term_id": "GO:0000976",
  "gene": "UniProtKB:Q17R98",
  "gene_symbol": "ZNF827",
  "term_label": "transcription cis-regulatory region binding",
  "gene_name": "Zinc finger protein 827"
}